xanthine biosynthetic process [GO:0046111] (biological process) Sources: GOC:go_curators Relationships: is a type of GO:0009113; is a type of xanthine metabolic process [GO:0046110] Definition: The chemical reactions and pathways resulting in the formation of xanthine, 2,6-dihydroxypurine, a purine formed in the metabolic breakdown of guanine but not present in nucleic acids. Also known as: xanthine anabolism, xanthine biosynthesis, xanthine formation, xanthine synthesis